{
  "gene_name": "Adenylate kinase 9",
  "gene": "UniProtKB:Q5TCS8",
  "term_label": "nucleus",
  "gene_symbol": "AK9",
  "term_id": "GO:0005634"
}